{
  "gene": "UniProtKB:P49137",
  "term_id": "GO:0048010",
  "term_label": "vascular endothelial growth factor receptor signaling pathway",
  "gene_symbol": "MAPKAPK2",
  "gene_name": "MAP kinase-activated protein kinase 2"
}